{
  "term_id": "GO:0005737",
  "gene": "UniProtKB:Q00169",
  "gene_symbol": "PITPNA",
  "term_label": "cytoplasm",
  "gene_name": "Phosphatidylinositol transfer protein alpha isoform"
}